{
  "term_label": "Unknown cellular component",
  "term_id": "UNKNOWN:0003",
  "gene_symbol": "TATDN1",
  "gene": "UniProtKB:Q6P1N9",
  "gene_name": "Deoxyribonuclease TATDN1"
}